positive regulation of xenobiotic detoxification by transmembrane export across the plasma membrane [GO:1905701] (biological process) Also known as: activation of drug transmembrane export, positive regulation of drug transmembrane export, positive regulation of xenobiotic transmembrane export, up regulation of drug transmembrane export, up-regulation of drug transmembrane export, upregulation of drug transmembrane export Relationships: is a type of positive regulation of transmembrane transport [GO:0034764]; is a type of positive regulation of response to stimulus [GO:0048584]; is a type of GO:1905699; positively regulates xenobiotic detoxification by transmembrane export across the plasma membrane [GO:1990961] Definition: Any process that activates or increases the frequency, rate or extent of xenobiotic transmembrane export. A xenobiotic is a compound foreign to the organism exposed to it. It may be synthesized by another organism (like ampicilin) or it can be a synthetic chemical. References: PMID:15198509 Sources: GOC:TermGenie, GOC:krc, GO_REF:0000058